regulation of superoxide dismutase activity [GO:1901668] (biological process) Definition: Any process that modulates the frequency, rate or extent of superoxide dismutase activity. Also known as: regulation of superoxide:superoxide oxidoreductase activity, regulation of Cu-Zn superoxide dismutase activity, regulation of Mn, Fe superoxide dismutase, regulation of copper, zinc superoxide dismutase activity, regulation of ferrisuperoxide dismutase activity, regulation of iron superoxide dismutase activity, regulation of manganese superoxide dismutase activity, regulation of nickel superoxide dismutase activity, regulation of Cu,Zn-SOD, regulation of Fe-SOD, regulation of Mn-SOD, regulation of SOD, regulation of SOD-1, regulation of SOD-2, regulation of SOD-3, regulation of SOD-4, regulation of SODF, regulation of SODS, regulation of cuprein, regulation of cytocuprein, regulation of erythrocuprein, regulation of hemocuprein, regulation of hepatocuprein, regulation of iron superoxide oxidoreductase, regulation of manganese superoxide oxidoreductase, regulation of nickel superoxide oxidoreductase, regulation of superoxide dismutase I, regulation of superoxide dismutase II, regulation of zinc superoxide oxidoreductase Sources: GOC:TermGenie Relationships: is_a regulation of oxidoreductase activity [GO:0051341]; regulates superoxide dismutase activity [GO:0004784] Subtypes: positive regulation of superoxide dismutase activity [GO:1901671]